{
  "gene": "UniProtKB:Q9UIF7",
  "gene_symbol": "MUTYH",
  "term_id": "GO:0000701",
  "term_label": "purine-specific mismatch base pair DNA N-glycosylase activity",
  "gene_name": "Adenine DNA glycosylase"
}